{
  "gene": "UniProtKB:P47992",
  "gene_name": "Lymphotactin",
  "term_label": "inflammatory response",
  "gene_symbol": "XCL1",
  "term_id": "GO:0006954"
}